{
  "term_label": "signal transduction",
  "term_id": "GO:0007165",
  "gene_name": "T-cell-interacting, activating receptor on myeloid cells protein 1",
  "gene_symbol": "TARM1",
  "gene": "UniProtKB:B6A8C7"
}